{
  "gene_symbol": "SERPINA2",
  "gene_name": "Alpha-1-antitrypsin-related protein",
  "gene": "UniProtKB:P20848",
  "term_id": "GO:0004867",
  "term_label": "serine-type endopeptidase inhibitor activity"
}